{
  "term_id": "GO:0006995",
  "gene_symbol": "ATG7",
  "gene_name": "Ubiquitin-like modifier-activating enzyme ATG7",
  "gene": "UniProtKB:O95352",
  "term_label": "cellular response to nitrogen starvation"
}